adenylate cyclase-inhibiting opioid receptor signaling pathway [GO:0031635] (biological process) Definition: An adenylate cyclase-inhibiting G protein-coupled receptor signaling pathway initiated by an opioid binding to its receptor, and ending with the regulation of a downstream cellular process. Also known as: opioid receptor, adenylate cyclase inhibiting pathway, inhibition of adenylate cyclase activity by opioid receptor signaling pathway, inhibition of adenylate cyclase activity by opioid receptor signalling pathway Sources: GOC:dph, GOC:mah, GOC:signaling, GOC:tb Regulation: regulated by regulation of adenylate cyclase-inhibiting opioid receptor signaling pathway [GO:1900729]; negatively regulated by negative regulation of adenylate cyclase-inhibiting opioid receptor signaling pathway [GO:1900730]; RO_0002213 by GO:1900731 Relationships: is a type of adenylate cyclase-inhibiting G protein-coupled receptor signaling pathway [GO:0007193]; is a type of G protein-coupled opioid receptor signaling pathway [GO:0038003]